basement membrane constituent secretion [GO:0061864] (biological process) Definition: The controlled release of molecules that form the basement membrane, including carbohydrates and glycoproteins by a cell. References: PMID:26610918, PMID:28228250 Relationships: is a type of extracellular matrix constituent secretion [GO:0070278] Subtypes: polarized secretion of basement membrane proteins in epithelium [GO:0061865]